inner medullary collecting duct development [GO:0072061] (biological process) Sources: GOC:mtg_kidney_jan10 Definition: The process whose specific outcome is the progression of the inner medullary collecting duct over time, from its formation to the mature structure. The inner medullary collecting duct is the portion of the collecting duct that lies in the renal inner medulla. Relationships: is a type of collecting duct development [GO:0072044]